{
  "gene_symbol": "CHD1",
  "gene_name": "Chromodomain-helicase-DNA-binding protein 1",
  "gene": "UniProtKB:O14646",
  "term_id": "GO:0034728",
  "term_label": "nucleosome organization"
}